{
  "gene": "UniProtKB:Q8IXI2",
  "term_label": "mitochondrion organization",
  "gene_name": "Mitochondrial Rho GTPase 1",
  "gene_symbol": "RHOT1",
  "term_id": "GO:0007005"
}